glomerular mesangial cell development [GO:0072144] (biological process) Sources: GOC:mtg_kidney_jan10 Definition: The process whose specific outcome is the progression of a glomerular mesangial cell in the kidney over time, from its formation to the mature structure. Relationships: is a type of GO:0002064; is_a GO:0072143; BFO_0000050 glomerular mesangial cell differentiation [GO:0072008] Subtypes: mesonephric glomerular mesangial cell development [GO:0061263], metanephric glomerular mesangial cell development [GO:0072255]